cellular response to cytokinin stimulus [GO:0071368] (biological process) Relationships: is a type of response to cytokinin [GO:0009735]; is a type of cellular response to hormone stimulus [GO:0032870] Sources: GOC:mah Definition: Any process that results in a change in state or activity of a cell (in terms of movement, secretion, enzyme production, gene expression, etc.) as a result of a cytokinin stimulus.